{
  "gene": "UniProtKB:Q8IWF9",
  "gene_name": "Coiled-coil domain-containing protein 83",
  "term_id": "UNKNOWN:0002",
  "term_label": "Unknown biological process",
  "gene_symbol": "CCDC83"
}